olfactory placode morphogenesis [GO:0071699] (biological process) Definition: The process in which the anatomical structures of the olfactory placode are generated and organized. The olfactory placode is a thickening of the neural ectoderm in the head region of the vertebrate embryo which develops into the olfactory region of the nasal cavity. Sources: GOC:mah Relationships: is a type of GO:0048598; is a type of ectodermal placode morphogenesis [GO:0071697]; is part of olfactory placode development [GO:0071698]